{
  "gene": "UniProtKB:Q9BYB0",
  "gene_name": "SH3 and multiple ankyrin repeat domains protein 3",
  "gene_symbol": "SHANK3",
  "term_id": "GO:0008306",
  "term_label": "associative learning"
}